{
  "gene_symbol": "DLL4",
  "gene_name": "Delta-like protein 4",
  "gene": "UniProtKB:Q9NR61",
  "term_id": "GO:0005112",
  "term_label": "Notch binding"
}